tyrosine-based site-specific recombinase activity [GO:0009037] (molecular function) Relationships: is a type of GO:0009009 Also known as: tyrosine recombinase, site-specific tyrosine recombinase activity Definition: Catalysis of the formation of new phosphodiester bonds between a pair of short, unique DNA target sequences; occurs through a phosphotyrosyl intermediate in which the target sequence is first cleaved by the nucleophilic attack by a tyrosine in the active site. References: PMID:11090626 Sources: GOC:elh